{
  "term_label": "cytoplasm",
  "gene_symbol": "IVNS1ABP",
  "gene_name": "Influenza virus NS1A-binding protein",
  "gene": "UniProtKB:Q9Y6Y0",
  "term_id": "GO:0005737"
}